{
  "gene": "UniProtKB:Q15628",
  "gene_symbol": "TRADD",
  "gene_name": "Tumor necrosis factor receptor type 1-associated DEATH domain protein",
  "term_label": "extrinsic apoptotic signaling pathway",
  "term_id": "GO:0097191"
}